{
  "gene_symbol": "HOXA3",
  "term_label": "embryonic skeletal system morphogenesis",
  "gene": "UniProtKB:O43365",
  "gene_name": "Homeobox protein Hox-A3",
  "term_id": "GO:0048704"
}